dihydropyrimidine dehydrogenase (NADP+) activity [GO:0017113] (molecular function) Definition: Catalysis of the reaction: 5,6-dihydrouracil + NADP+ = uracil + NADPH + H+. Sources: EC:1.3.1.2 Also known as: dihydropyrimidine dehydrogenase activity, 4,5-dihydrothymine: oxidoreductase activity, 5,6-dihydrouracil:NADP+ 5-oxidoreductase activity, DHPDH, DHU dehydrogenase activity, DPD, dehydrogenase, dihydrouracil (nicotinamide adenine dinucleotide phosphate), dihydrothymine dehydrogenase activity, dihydrouracil dehydrogenase (NADP), dihydrouracil dehydrogenase (NADP+) activity, hydropyrimidine dehydrogenase activity Relationships: is a type of GO:0016628